{
  "gene_symbol": "ADCYAP1R1",
  "gene_name": "Pituitary adenylate cyclase-activating polypeptide type I receptor",
  "gene": "UniProtKB:P41586",
  "term_label": "G protein-coupled peptide receptor activity",
  "term_id": "GO:0008528"
}